{
  "gene": "UniProtKB:P78334",
  "term_label": "gamma-aminobutyric acid signaling pathway",
  "term_id": "GO:0007214",
  "gene_symbol": "GABRE",
  "gene_name": "Gamma-aminobutyric acid receptor subunit epsilon"
}